positive regulation of G protein-coupled receptor internalization [GO:1904022] (biological process) Also known as: positive regulation of G-protein coupled receptor internalization, up regulation of G-protein coupled receptor internalization, up-regulation of G-protein coupled receptor internalization, upregulation of G-protein coupled receptor internalization, activation of G-protein coupled receptor internalization References: PMID:24732013 Sources: GOC:TermGenie, GO_REF:0000058 Relationships: is a type of GO:0002092; is a type of regulation of G protein-coupled receptor internalization [GO:1904020]; RO_0002213 G protein-coupled receptor internalization [GO:0002031] Definition: Any process that activates or increases the frequency, rate or extent of G protein-coupled receptor internalization.